chromatin organization [GO:0006325] (biological process) Definition: The assembly or remodeling of chromatin composed of DNA complexed with histones, other associated proteins, and sometimes RNA. Relationships: is a type of cellular component organization [GO:0016043] Subtypes: DNA replication-dependent chromatin assembly [GO:0006335], GO:0006338, GO:0034080, sperm DNA decondensation [GO:0035041], sperm DNA condensation [GO:0035092], GO:0070828, chromatin looping [GO:0140588], DNA replication-dependent chromatin disassembly [GO:0140889], chromosomal DNA methylation maintenance following DNA replication [GO:0141119], nucleolar chromatin organization [GO:1990700] Regulation: regulated by GO:1902275; negatively regulated by negative regulation of chromatin organization [GO:1905268]; positively regulated by positive regulation of chromatin organization [GO:1905269] References: PMID:20404130 Also known as: chromatin maintenance, chromatin organisation, establishment of chromatin architecture, establishment or maintenance of chromatin architecture, DNA replication-independent chromatin assembly, DNA replication-independent chromatin organization, DNA replication-independent nucleosome organisation, DNA replication-independent nuclesome assembly, chromatin assembly, transcription-coupled nucleosome assembly, chromatin assembly or disassembly, chromatin assembly/disassembly, chromatin modification